L,L-diaminopimelate aminotransferase activity [GO:0010285] (molecular function) Definition: Catalysis of the reaction: 2-oxoglutarate + LL-2,6-diaminopimelate = (S)-2,3,4,5-tetrahydrodipicolinate + L-glutamate + H2O + H+. Relationships: is a type of transaminase activity [GO:0008483] Sources: EC:2.6.1.83, RHEA:23988 Also known as: LL-2,6-diaminoheptanedioate:2-oxoglutarate aminotransferase activity, LL-diaminopimelate aminotransferase activity, LL-DAP aminotransferase activity, LL-DAP-AT activity, LL-diaminopimelate transaminase activity